{
  "term_label": "Unknown cellular component",
  "term_id": "UNKNOWN:0003",
  "gene_name": "Putative protein FAM90A8",
  "gene_symbol": "FAM90A8",
  "gene": "UniProtKB:A6NJQ4"
}